{
  "gene_name": "Forkhead box protein L2",
  "term_id": "GO:0030154",
  "gene": "UniProtKB:P58012",
  "gene_symbol": "FOXL2",
  "term_label": "cell differentiation"
}